{
  "term_id": "GO:0008104",
  "gene": "UniProtKB:Q8IYM1",
  "term_label": "intracellular protein localization",
  "gene_symbol": "SEPTIN12",
  "gene_name": "Septin-12"
}